{
  "gene_name": "Arginase-2, mitochondrial",
  "term_id": "GO:0005739",
  "gene_symbol": "ARG2",
  "gene": "UniProtKB:P78540",
  "term_label": "mitochondrion"
}